jasmonoyl-L-amino acid ligase activity [GO:0080123] (molecular function) Also known as: ja-amino synthetase activity, jasmonate-amido synthetase activity, jasmonate-amino acid conjugate synthetase activity, jasmonate-amino acid synthetase activity, jasmonate-amino synthetase activity, jasmonate:amino acid synthetase activity, jasmonic acid-amino synthetase activity, jasmonyl-amino synthetase activity Definition: Catalysis of the reaction: a jasmonate + an L-alpha-amino acid + ATP = a jasmonyl-L-amino acid + AMP + diphosphate + H+. In Arabidopsis, isoleucine is the principal amino acid that conjugates with JA to form JA (JA-Ile). Other amino acid can be conjugated with JA such as valine, leucine, and phenylalanine. References: PMID:15258265, PMID:17291501, PMID:33821356 Sources: RHEA:55772 Relationships: is a type of acid-amino acid ligase activity [GO:0016881]